phthalyl amidase activity [GO:0047418] (molecular function) Also known as: o-phthalyl amidase activity, phthalyl-amide amidohydrolase activity Relationships: is_a GO:0016811 Sources: EC:3.5.1.79, MetaCyc:3.5.1.79-RXN Definition: Catalysis of the reaction: H2O + a phthalylamide = phthalate + substituted amine.